{
  "term_label": "mitotic DNA replication checkpoint signaling",
  "gene_name": "Zinc finger protein 830",
  "gene": "UniProtKB:Q96NB3",
  "term_id": "GO:0033314",
  "gene_symbol": "ZNF830"
}